{
  "gene_symbol": "STUB1",
  "gene_name": "E3 ubiquitin-protein ligase CHIP",
  "term_id": "GO:0061630",
  "term_label": "ubiquitin protein ligase activity",
  "gene": "UniProtKB:Q9UNE7"
}